{
  "term_id": "UNKNOWN:0001",
  "gene_name": "Tetraspanin-14",
  "term_label": "Unknown molecular function",
  "gene_symbol": "TSPAN14",
  "gene": "UniProtKB:Q8NG11"
}